{
  "gene_name": "tRNA endonuclease ANKZF1",
  "gene_symbol": "ANKZF1",
  "term_label": "Unknown cellular component",
  "gene": "UniProtKB:Q9H8Y5",
  "term_id": "UNKNOWN:0003"
}